positive regulation of natural killer cell degranulation [GO:0043323] (biological process) Also known as: positive regulation of NK cell degranulation, positive regulation of NK cell granule exocytosis, positive regulation of natural killer cell granule exocytosis, up regulation of natural killer cell degranulation, up-regulation of natural killer cell degranulation, upregulation of natural killer cell degranulation, activation of natural killer cell degranulation, stimulation of natural killer cell degranulation Sources: ISBN:0781735149 Relationships: is a type of positive regulation of leukocyte degranulation [GO:0043302]; is a type of regulation of natural killer cell degranulation [GO:0043321]; is a type of positive regulation of natural killer cell mediated cytotoxicity [GO:0045954]; positively regulates natural killer cell degranulation [GO:0043320] Definition: Any process that activates or increases the frequency, rate or extent of natural killer cell degranulation.